molybdopterin synthase activity [GO:0030366] (molecular function) References: PMID:18154309, PMID:8514783 Definition: Catalysis of the conversion of precursor Z to molybdopterin, the final step in molybdopterin biosynthesis. Relationships: is a type of GO:0016783